{
  "term_id": "GO:0005634",
  "gene": "UniProtKB:Q15784",
  "term_label": "nucleus",
  "gene_symbol": "NEUROD2",
  "gene_name": "Neurogenic differentiation factor 2"
}